{
  "gene_symbol": "ANGPTL2",
  "term_id": "UNKNOWN:0002",
  "gene": "UniProtKB:Q9UKU9",
  "gene_name": "Angiopoietin-related protein 2",
  "term_label": "Unknown biological process"
}